{
  "term_id": "GO:0006414",
  "gene_symbol": "EIF5A",
  "gene_name": "Eukaryotic translation initiation factor 5A-1",
  "term_label": "translational elongation",
  "gene": "UniProtKB:P63241"
}